positive regulation of protein import [GO:1904591] (biological process) References: PMID:11406629 Sources: GOC:TermGenie, GO_REF:0000058 Relationships: is a type of positive regulation of protein transport [GO:0051222]; is a type of regulation of protein import [GO:1904589]; positively regulates GO:0017038 Also known as: positive regulation of protein uptake, up regulation of protein import, up regulation of protein uptake, up-regulation of protein import, up-regulation of protein uptake, upregulation of protein import, upregulation of protein uptake, activation of protein import, activation of protein uptake Definition: Any process that activates or increases the frequency, rate or extent of protein import.